negative regulation of neutrophil migration [GO:1902623] (biological process) Also known as: down regulation of neutrophil migration, down-regulation of neutrophil migration, downregulation of neutrophil migration, inhibition of neutrophil migration References: PMID:1826836 Sources: GOC:TermGenie, GO_REF:0000058 Relationships: is a type of negative regulation of leukocyte migration [GO:0002686]; is a type of GO:1902622; negatively regulates neutrophil migration [GO:1990266] Definition: Any process that stops, prevents or reduces the frequency, rate or extent of neutrophil migration. Subtypes: GO:0090024, GO:2000390